{
  "gene": "UniProtKB:P03999",
  "gene_symbol": "OPN1SW",
  "gene_name": "Short-wave-sensitive opsin 1",
  "term_label": "G protein-coupled photoreceptor activity",
  "term_id": "GO:0008020"
}